{
  "term_id": "GO:0032511",
  "term_label": "late endosome to vacuole transport via multivesicular body sorting pathway",
  "gene": "UniProtKB:O95807",
  "gene_name": "Transmembrane protein 50A",
  "gene_symbol": "TMEM50A"
}